{
  "gene_symbol": "TIFAB",
  "gene_name": "TRAF-interacting protein with FHA domain-containing protein B",
  "gene": "UniProtKB:Q6ZNK6",
  "term_id": "UNKNOWN:0003",
  "term_label": "Unknown cellular component"
}